{
  "gene_name": "Guanylate cyclase activator 2B",
  "term_label": "guanylate cyclase activator activity",
  "gene_symbol": "GUCA2B",
  "gene": "UniProtKB:Q16661",
  "term_id": "GO:0030250"
}